{
  "gene_name": "Polyribonucleotide nucleotidyltransferase 1, mitochondrial",
  "term_id": "GO:0005739",
  "term_label": "mitochondrion",
  "gene": "UniProtKB:Q8TCS8",
  "gene_symbol": "PNPT1"
}